histone H3T11 kinase activity [GO:0035402] (molecular function) Also known as: histone H3-T11 kinase activity, histone kinase activity (H3-T11 specific), histone threonine kinase activity (H3-T11 specific), histone-threonine kinase activity (H3-T11 specific) Relationships: is a type of protein serine/threonine kinase activity [GO:0004674]; is a type of GO:0140996 Sources: GOC:bf Note: Comment: Note that the residue position corresponds to the canonical human H3 histone (UniProtKB:P84243); this residue is conserved across all eukaryotes. Residue 1 is the first residue following removal of the initiating Methionine (Met). Note that each histone is encoded by multiple genes, and sequences may vary across different genes within an organism. Definition: Catalysis of the reaction: histone H3-threonine (position 11) + ATP = histone H3-phosphothreonine (position 11) + ADP. This reaction is the addition of a phosphate group to the threonine residue at position 11 of histone H3.